3-hydroxyphenyl propanoate transport [GO:0015731] (biological process) Relationships: is a type of organic hydroxy compound transport [GO:0015850] Also known as: 3-hydroxyphenyl propionate transport Sources: GOC:krc Definition: The directed movement of 3-hydroxyphenyl propanoate into, out of or within a cell, or between cells, by means of some agent such as a transporter or pore.